epithelial cell-cell adhesion involved in epithelium migration [GO:0090137] (BP) Definition: The attachment of an epithelial cell to another epithelial cell via adhesion molecules that contributes to epithelium migration. Relationships: is a type of epithelial cell-cell adhesion [GO:0090136]; is part of GO:0090132 Sources: GOC:ascb_2009, GOC:dph, GOC:tb Regulation: regulated by regulation of epithelial cell-cell adhesion involved in epithelium migration [GO:1903681]; negatively regulated by negative regulation of epithelial cell-cell adhesion involved in epithelium migration [GO:1903682]; positively regulated by positive regulation of epithelial cell-cell adhesion involved in epithelium migration [GO:1903683]